{
  "term_label": "nervous system development",
  "gene_symbol": "LDB2",
  "gene": "UniProtKB:O43679",
  "term_id": "GO:0007399",
  "gene_name": "LIM domain-binding protein 2"
}